{
  "term_id": "UNKNOWN:0002",
  "gene_symbol": "FAM236B",
  "term_label": "Unknown biological process",
  "gene": "UniProtKB:A0A1B0GV22",
  "gene_name": "Protein FAM236B"
}